{
  "term_label": "RNA binding",
  "gene": "UniProtKB:Q7Z417",
  "gene_name": "FMR1-interacting protein NUFIP2",
  "term_id": "GO:0003723",
  "gene_symbol": "NUFIP2"
}